{
  "gene_name": "Testin",
  "gene_symbol": "TES",
  "term_id": "UNKNOWN:0001",
  "term_label": "Unknown molecular function",
  "gene": "UniProtKB:Q9UGI8"
}